{
  "gene": "UniProtKB:Q9Y6N8",
  "term_id": "GO:0099560",
  "gene_name": "Cadherin-10",
  "term_label": "synaptic membrane adhesion",
  "gene_symbol": "CDH10"
}